{
  "gene": "UniProtKB:P0DPI2",
  "term_id": "GO:0005739",
  "gene_symbol": "GATD3",
  "term_label": "mitochondrion",
  "gene_name": "Glutamine amidotransferase-like class 1 domain-containing protein 3, mitochondrial"
}